{
  "term_label": "regulation of vasculogenesis",
  "gene": "UniProtKB:Q92556",
  "gene_name": "Engulfment and cell motility protein 1",
  "gene_symbol": "ELMO1",
  "term_id": "GO:2001212"
}